{
  "gene": "UniProtKB:Q05BV3",
  "term_label": "Unknown cellular component",
  "gene_name": "Echinoderm microtubule-associated protein-like 5",
  "gene_symbol": "EML5",
  "term_id": "UNKNOWN:0003"
}